{
  "term_label": "microfilament motor activity",
  "gene_name": "Myosin-7",
  "gene": "UniProtKB:P12883",
  "gene_symbol": "MYH7",
  "term_id": "GO:0000146"
}